regulation of TORC2 signaling [GO:1903939] (biological process) Definition: Any process that modulates the frequency, rate or extent of TORC2 signaling. Relationships: is a type of GO:0032006; regulates GO:0038203 Also known as: regulation of TORC2 signal transduction Subtypes: negative regulation of TORC2 signaling [GO:1903940], GO:1904515 References: PMID:24247430 Sources: GOC:TermGenie, GO_REF:0000058